chemoattraction of branchiomotor neuron axon in neural tube [GO:0021788] (biological process) Also known as: positive chemotaxis of branchiomotor neuron axon in neural tube Relationships: is a type of branchiomotor neuron axon guidance in neural tube [GO:0021786]; is a type of chemoattraction of branchiomotor axon [GO:0021792] Definition: The process in which a branchiomotor neuron growth cone in the neural tube is directed to a specific target site in the neural tube in response to an attractive chemical cue. Branchiomotor neurons are located in the hindbrain and innervate branchial arch-derived muscles that control jaw movements, facial expression, the larynx, and the pharynx. References: PMID:14699587 Sources: GOC:cls, GOC:dgh, GOC:dph, GOC:jid, GO_REF:0000021